{
  "gene_name": "rRNA N6-adenosine-methyltransferase METTL5",
  "term_id": "GO:0008988",
  "gene_symbol": "METTL5",
  "term_label": "rRNA (adenine-N6-)-methyltransferase activity",
  "gene": "UniProtKB:Q9NRN9"
}